gluconate import across plasma membrane [GO:0140270] (biological process) Definition: The directed movement of gluconate from outside of a cell, across the plasma membrane and into the cytosol. References: PMID:10735857 Relationships: is a type of gluconate transmembrane transport [GO:0035429]; is a type of import across plasma membrane [GO:0098739]